{
  "gene": "UniProtKB:Q9Y4X3",
  "gene_symbol": "CCL27",
  "term_id": "GO:0006954",
  "term_label": "inflammatory response",
  "gene_name": "C-C motif chemokine 27"
}